uracil transport [GO:0015857] (biological process) Sources: GOC:go_curators Definition: The directed movement of uracil, 2,4-dioxopyrimidine, into, out of or within a cell, or between cells, by means of some agent such as a transporter or pore. Relationships: is a type of GO:0015855 Subtypes: uracil transmembrane transport [GO:1903791]